sulfur utilization [GO:0006791] (biological process) Regulation: regulated by regulation of sulfur utilization [GO:0006792]; negatively regulated by negative regulation of sulfur utilization [GO:0045882]; positively regulated by positive regulation of sulfur utilization [GO:0045883] Sources: GOC:mah, GOC:mlg Definition: A series of processes that forms an integrated mechanism by which a cell or an organism detects the depletion of primary sulfur sources and then activates genes to scavenge the last traces of the primary sulfur source and to transport and metabolize alternate sulfur sources. The utilization process begins when the cell or organism detects sulfur levels, includes the activation of genes whose products detect, transport or metabolize sulfur-containing compounds, and ends when the sulfur is incorporated into the cell or organism's metabolism. Also known as: sulphur utilization Relationships: is a type of response to nutrient levels [GO:0031667]; has part GO:0006790; has part sulfur compound transport [GO:0072348]